constitutive protein ectodomain proteolysis [GO:0051089] (biological process) Definition: The proteolytic cleavage of transmembrane proteins and release of their ectodomain that occurs constantly, regardless of environmental conditions or demands. References: PMID:12714508 Relationships: is a type of membrane protein ectodomain proteolysis [GO:0006509]